{
  "gene": "UniProtKB:Q99470",
  "gene_symbol": "SDF2",
  "gene_name": "Stromal cell-derived factor 2",
  "term_label": "Unknown cellular component",
  "term_id": "UNKNOWN:0003"
}